{
  "term_id": "UNKNOWN:0001",
  "gene": "UniProtKB:Q8IZJ3",
  "gene_name": "C3 and PZP-like alpha-2-macroglobulin domain-containing protein 8",
  "term_label": "Unknown molecular function",
  "gene_symbol": "CPAMD8"
}